regulation of fertilization [GO:0080154] (biological process) References: PMID:20478994 Sources: GOC:DHL Definition: Any process that modulates the rate, frequency or extent of fertilization. Fertilization is the union of gametes of opposite sexes during the process of sexual reproduction to form a zygote. It involves the fusion of the gametic nuclei (karyogamy) and cytoplasm (plasmogamy). Relationships: is a type of GO:2000241; regulates fertilization [GO:0009566] Subtypes: GO:0060467, GO:0080155, positive regulation of fertilization [GO:1905516]